{
  "gene_name": "Cerebellin-1",
  "term_label": "maintenance of synapse structure",
  "gene_symbol": "CBLN1",
  "term_id": "GO:0099558",
  "gene": "UniProtKB:P23435"
}